{
  "gene": "UniProtKB:O14492",
  "gene_symbol": "SH2B2",
  "term_id": "GO:0035556",
  "gene_name": "SH2B adapter protein 2",
  "term_label": "intracellular signal transduction"
}